{
  "term_id": "GO:0033344",
  "gene_name": "Apolipoprotein M",
  "gene": "UniProtKB:O95445",
  "gene_symbol": "APOM",
  "term_label": "cholesterol efflux"
}